endoplasmic reticulum organization [GO:0007029] (biological process) Relationships: is a type of organelle organization [GO:0006996]; is part of endomembrane system organization [GO:0010256] Subtypes: GO:0016320, vesicle fusion with endoplasmic reticulum [GO:0048279], endoplasmic reticulum inheritance [GO:0048309], GO:0061163, endoplasmic reticulum cisternal network organization [GO:0071783], endoplasmic reticulum tubular network organization [GO:0071786], endoplasmic reticulum disassembly [GO:1905692] Also known as: ER organisation, endoplasmic reticulum organisation, ER organization and biogenesis, endoplasmic reticulum morphology, endoplasmic reticulum organization and biogenesis Sources: GOC:dph, GOC:jl, GOC:mah Definition: A process that is carried out at the cellular level which results in the assembly, arrangement of constituent parts, or disassembly of the endoplasmic reticulum.